{
  "gene": "UniProtKB:Q9UK10",
  "term_label": "regulation of transcription by RNA polymerase II",
  "gene_symbol": "ZNF225",
  "gene_name": "Zinc finger protein 225",
  "term_id": "GO:0006357"
}